{
  "gene_symbol": "ELL",
  "gene": "UniProtKB:P55199",
  "term_id": "GO:0042795",
  "gene_name": "RNA polymerase II elongation factor ELL",
  "term_label": "snRNA transcription by RNA polymerase II"
}